{
  "gene": "UniProtKB:Q96FZ5",
  "gene_name": "CKLF-like MARVEL transmembrane domain-containing protein 7",
  "term_label": "Unknown molecular function",
  "term_id": "UNKNOWN:0001",
  "gene_symbol": "CMTM7"
}